{
  "gene": "UniProtKB:P21397",
  "term_id": "GO:0019607",
  "term_label": "phenylethylamine catabolic process",
  "gene_symbol": "MAOA",
  "gene_name": "Amine oxidase [flavin-containing] A"
}